{
  "gene_symbol": "POFUT2",
  "term_label": "Unknown cellular component",
  "term_id": "UNKNOWN:0003",
  "gene_name": "GDP-fucose protein O-fucosyltransferase 2",
  "gene": "UniProtKB:Q9Y2G5"
}